{
  "term_label": "plasma membrane",
  "gene": "UniProtKB:Q9NYQ6",
  "gene_name": "Cadherin EGF LAG seven-pass G-type receptor 1",
  "gene_symbol": "CELSR1",
  "term_id": "GO:0005886"
}